peripheral nervous system neuron development [GO:0048935] (biological process) Sources: GOC:dgh Definition: The process whose specific outcome is the progression of a neuron whose cell body is located in the peripheral nervous system, from initial commitment of the cell to a neuronal fate, to the fully functional differentiated neuron. Subtypes: GO:0060959 Relationships: is_a GO:0048666; is part of peripheral nervous system neuron differentiation [GO:0048934]